{
  "gene_name": "SLAIN motif-containing protein 2",
  "term_label": "cytoplasmic microtubule organization",
  "term_id": "GO:0031122",
  "gene": "UniProtKB:Q9P270",
  "gene_symbol": "SLAIN2"
}